{
  "gene_name": "Olfactory receptor 10W1",
  "term_id": "GO:0004984",
  "term_label": "olfactory receptor activity",
  "gene_symbol": "OR10W1",
  "gene": "UniProtKB:Q8NGF6"
}